high-density lipoprotein particle [GO:0034364] (cellular component) Definition: A lipoprotein particle with a high density (typically 1.063-1.21 g/ml) and a diameter of 5-10 nm that contains APOAs and may contain APOCs and APOE; found in blood and carries lipids from body tissues to the liver as part of the reverse cholesterol transport process. Sources: GOC:BHF, GOC:expert_pt, GOC:mah, GOC:pde, GOC:rl Also known as: HDL complex, HDL particle, high-density lipoprotein class complex, HDL2, HDL3 Relationships: is a type of GO:0034358 Subtypes: GO:0034365, GO:0034366